{
  "gene_name": "Germinal-center associated nuclear protein",
  "term_id": "GO:0070390",
  "gene": "UniProtKB:O60318",
  "term_label": "transcription export complex 2",
  "gene_symbol": "MCM3AP"
}